{
  "term_label": "Unknown molecular function",
  "gene_symbol": "RASSF5",
  "term_id": "UNKNOWN:0001",
  "gene_name": "Ras association domain-containing protein 5",
  "gene": "UniProtKB:Q8WWW0"
}